{
  "gene_symbol": "DTNBP1",
  "gene": "UniProtKB:Q96EV8",
  "gene_name": "Dysbindin",
  "term_label": "regulation of synaptic vesicle exocytosis",
  "term_id": "GO:2000300"
}